glutamate synthase (NADPH) activity [GO:0004355] (molecular function) Sources: EC:1.4.1.13, RHEA:15501 Also known as: GOGAT activity, L-glutamate synthase activity, L-glutamate synthetase activity, NADPH GOGAT, L-glutamate:NADP+ oxidoreductase (transaminating), L-glutamine:2-oxoglutarate aminotransferase, NADPH oxidizing activity, NADPH-dependent glutamate synthase activity, NADPH-glutamate synthase activity, NADPH-linked glutamate synthase, glutamate (reduced nicotinamide adenine dinucleotide phosphate) synthase activity, glutamate synthetase (NADP) activity, glutamine amide-2-oxoglutarate aminotransferase (oxidoreductase, NADP) activity, glutamine-ketoglutaric aminotransferase activity Note: Note that this term has a MetaCyc pathway reference as the pathway only has a single step. Relationships: is a type of GO:0015930 Definition: Catalysis of the reaction: 2 L-glutamate + NADP+ = 2-oxoglutarate + L-glutamine + H+ + NADPH. This is a two-step reaction: (a) L-glutamate + NH3 = L-glutamine + H2O, (b) L-glutamate + NADP+ + H2O = NH3 + 2-oxoglutarate + NADPH + H+.